{
  "gene_symbol": "HASPIN",
  "term_label": "histone H3T3 kinase activity",
  "term_id": "GO:0072354",
  "gene": "UniProtKB:Q8TF76",
  "gene_name": "Serine_threonine-protein kinase haspin"
}